{
  "term_id": "GO:0005829",
  "gene_symbol": "AS3MT",
  "gene_name": "Arsenite methyltransferase",
  "term_label": "cytosol",
  "gene": "UniProtKB:Q9HBK9"
}